{
  "term_label": "extracellular space",
  "gene": "UniProtKB:P09038",
  "gene_name": "Fibroblast growth factor 2",
  "gene_symbol": "FGF2",
  "term_id": "GO:0005615"
}